{
  "term_id": "GO:0005615",
  "gene_symbol": "WNT4",
  "gene": "UniProtKB:P56705",
  "term_label": "extracellular space",
  "gene_name": "Protein Wnt-4"
}